polar nucleus fusion [GO:0010197] (biological process) Definition: The merging of the polar nuclei, the two nuclei contained within the same cell that are created from the mitotic division of the megaspore during angiosperm reproduction. Polar nuclear fusion takes place in the ovule, forming in the fusion nucleus and giving rise to the endosperm when fertilized. Relationships: is_a karyogamy [GO:0000741]; BFO_0000050 GO:0009559 Sources: GOC:mtg_plant, GOC:sm